{
  "gene": "UniProtKB:Q6P1J6",
  "term_label": "phospholipid metabolic process",
  "gene_name": "Phospholipase B1, membrane-associated",
  "gene_symbol": "PLB1",
  "term_id": "GO:0006644"
}